forward locomotion [GO:0043056] (biological process) Definition: Anterior movement of an organism, following the direction of the head of the animal. Regulation: regulated by GO:0043059; negatively regulated by negative regulation of forward locomotion [GO:1905849]; positively regulated by GO:1905850 Relationships: is a type of directional locomotion [GO:0033058] Sources: GOC:go_curators